{
  "gene_name": "Survival of motor neuron-related-splicing factor 30",
  "term_label": "RNA binding",
  "gene": "UniProtKB:O75940",
  "gene_symbol": "SMNDC1",
  "term_id": "GO:0003723"
}